tRNA-intron endonuclease complex [GO:0000214] (cellular component) Also known as: SEN complex, tRNA splicing endonuclease complex Definition: A protein complex that catalyzes the endonucleolytic cleavage of pre-tRNA, producing 5'-hydroxyl and 2',3'-cyclic phosphate termini, and specifically removing the intron. Relationships: is a type of nuclear protein-containing complex [GO:0140513]; is a type of endoribonuclease complex [GO:1902555] References: PMID:22391451